ERBB4-ERBB4 complex [GO:0038141] (cellular component) Definition: A homodimeric complex containing two monomers of the tyrosine kinase receptor ERBB4 (also called HER4). References: PMID:16460914 Sources: GOC:signaling Also known as: ERBB4 homodimer Relationships: is_a plasma membrane signaling receptor complex [GO:0098802]